{
  "gene_symbol": "ADPRS",
  "gene_name": "ADP-ribosylhydrolase ARH3",
  "term_id": "GO:0140292",
  "term_label": "ADP-ribosylserine hydrolase activity",
  "gene": "UniProtKB:Q9NX46"
}